{
  "term_id": "GO:0005634",
  "term_label": "nucleus",
  "gene_name": "cAMP-dependent protein kinase catalytic subunit beta",
  "gene_symbol": "PRKACB",
  "gene": "UniProtKB:P22694"
}